{
  "gene_name": "Homeobox protein Hox-C5",
  "gene_symbol": "HOXC5",
  "term_label": "nucleus",
  "term_id": "GO:0005634",
  "gene": "UniProtKB:Q00444"
}